1-phosphatidylinositol-3-phosphate 4-kinase activity [GO:0052811] (molecular function) Relationships: is a type of phosphatidylinositol kinase activity [GO:0052742] Definition: Catalysis of the reaction: a 1-phosphatidyl-1D-myo-inositol 3-phosphate + ATP = a 1-phosphatidyl-1D-myo-inositol 3,4-bisphosphate + ADP + H+. References: PMID:9211928, PMID:9367159, PMID:9660759 Sources: RHEA:63688 Also known as: phosphatidylinositol 3-phosphate 4-kinase activity